{
  "gene_name": "Calsyntenin-1",
  "gene": "UniProtKB:O94985",
  "term_label": "postsynaptic density membrane",
  "term_id": "GO:0098839",
  "gene_symbol": "CLSTN1"
}